leg disc development [GO:0035218] (biological process) Definition: Progression of the leg imaginal disc over time, from its initial formation through to its metamorphosis to form adult structures including the leg, coxa and ventral thoracic pleura. Sources: GOC:bf, ISBN:0879694238 Relationships: is a type of GO:0007444